{
  "gene_symbol": "NR3C2",
  "gene_name": "Mineralocorticoid receptor",
  "term_id": "GO:0000785",
  "term_label": "chromatin",
  "gene": "UniProtKB:P08235"
}